{
  "term_id": "GO:0005794",
  "gene_symbol": "ZDHHC16",
  "gene": "UniProtKB:Q969W1",
  "gene_name": "Palmitoyltransferase ZDHHC16",
  "term_label": "Golgi apparatus"
}